valine-pyruvate transaminase activity [GO:0009042] (molecular function) Relationships: is a type of transaminase activity [GO:0008483] Definition: Catalysis of the reaction: L-valine + pyruvate = 3-methyl-2-oxobutanoate + L-alanine. Also known as: valine-pyruvate aminotransferase activity, transaminase C activity, L-valine:pyruvate aminotransferase activity, alanine--valine transaminase activity, alanine-oxoisovalerate aminotransferase activity, valine--pyruvate aminotransferase activity Sources: EC:2.6.1.66, RHEA:22912